{
  "term_id": "GO:0005886",
  "term_label": "plasma membrane",
  "gene_name": "CD151 antigen",
  "gene_symbol": "CD151",
  "gene": "UniProtKB:P48509"
}